{
  "term_id": "GO:0010273",
  "gene_name": "Metallothionein-3",
  "gene_symbol": "MT3",
  "gene": "UniProtKB:P25713",
  "term_label": "detoxification of copper ion"
}